regulation of xylose catabolic process to ethanol [GO:1900515] (biological process) Also known as: regulation of xylose catabolism to ethanol Relationships: is a type of regulation of fermentation [GO:0043465]; is a type of regulation of D-xylose catabolic process [GO:0043469]; regulates D-xylose catabolic process to ethanol [GO:0044577] Subtypes: negative regulation of xylose catabolic process to ethanol [GO:1900516], positive regulation of xylose catabolic process to ethanol [GO:1900517] Sources: GOC:TermGenie, GOC:mengo_curators Definition: Any process that modulates the frequency, rate or extent of xylose catabolic process to ethanol.